{
  "gene": "UniProtKB:Q8NGV5",
  "gene_symbol": "OR13D1",
  "gene_name": "Olfactory receptor 13D1",
  "term_label": "plasma membrane",
  "term_id": "GO:0005886"
}